autophagosome localization [GO:0061906] (biological process) References: PMID:26763909 Relationships: is a type of vacuolar localization [GO:1990849] Subtypes: autophagosome-dependent secretion [GO:0160192] Definition: Any process in which an autophagosome is transported to, and/or maintained in, a specific location within the cell.